posterior lateral line nerve glial cell differentiation [GO:0048931] (biological process) Relationships: is a type of lateral line nerve glial cell differentiation [GO:0048895]; is part of posterior lateral line nerve development [GO:0048918] Definition: The process in which a relatively unspecialized cell acquires specialized features of a glial cell in the posterior lateral line nerve. References: PMID:15832385